mitochondrial RNA polymerase general transcription initiation factor activity [GO:0180066] (molecular function) Definition: A general transcription initiation factor activity that contributes to transcription start site selection and transcription initiation by the mitochondrial RNA polymerase. References: PMID:29149603 Relationships: is a type of general transcription initiation factor activity [GO:0140223]